{
  "term_label": "phosphatidylcholine-retinol O-acyltransferase activity",
  "gene": "UniProtKB:O95237",
  "term_id": "GO:0047173",
  "gene_symbol": "LRAT",
  "gene_name": "Lecithin retinol acyltransferase"
}